penicillin biosynthetic process [GO:0042318] (biological process) Sources: GOC:jl, ISBN:0198506732 Also known as: penicillin anabolism, penicillin biosynthesis, penicillin formation, penicillin synthesis Relationships: is a type of beta-lactam antibiotic biosynthetic process [GO:0030654]; is a type of GO:0042316; is a type of GO:0044272; is_a secondary metabolite biosynthetic process [GO:0044550]; is a type of monocarboxylic acid biosynthetic process [GO:0072330] Definition: The chemical reactions and pathways resulting in the formation of any antibiotic that contains the condensed beta-lactamthiazolidine ring system. Subtypes: GO:1901088 Regulation: regulated by GO:1900196; negatively regulated by GO:1900197; positively regulated by positive regulation of penicillin biosynthetic process [GO:1900198]